regulation of postsynaptic neurotransmitter receptor diffusion trapping [GO:0150054] (BP) References: PMID:20935643 Sources: GOC:aruk, GOC:bc Relationships: is a type of regulation of cellular localization [GO:0060341]; is a type of regulation of biological quality [GO:0065008]; is a type of regulation of receptor localization to synapse [GO:1902683]; regulates postsynaptic neurotransmitter receptor diffusion trapping [GO:0098970] Definition: Any process that modulates the frequency, rate or extent of postsynaptic neurotransmitter receptor diffusion trapping.